{
  "gene_name": "SNF-related serine_threonine-protein kinase",
  "gene": "UniProtKB:Q9NRH2",
  "gene_symbol": "SNRK",
  "term_label": "Unknown biological process",
  "term_id": "UNKNOWN:0002"
}